ferric-chelate reductase (NADPH) activity [GO:0052851] (molecular function) Also known as: ferric chelate reductase activity, iron chelate reductase activity, ferric reductase, NADPH-dependent activity Definition: Catalysis of the reaction: 2 a Fe(II)-siderophore + NADP+ + H+ = 2 a Fe(III)-siderophore + NADPH. Sources: RHEA:28795 Relationships: is a type of ferric-chelate reductase activity [GO:0000293]; is a type of oxidoreductase activity, acting on metal ions, NAD or NADP as acceptor [GO:0016723]